{
  "term_label": "signaling adaptor activity",
  "gene_symbol": "NCK1",
  "term_id": "GO:0035591",
  "gene_name": "Cytoplasmic protein NCK1",
  "gene": "UniProtKB:P16333"
}